{
  "gene_name": "Histone H2A.V",
  "gene": "UniProtKB:Q71UI9",
  "term_label": "nucleosome",
  "term_id": "GO:0000786",
  "gene_symbol": "H2AZ2"
}